{
  "gene": "UniProtKB:P04818",
  "term_label": "cytosol",
  "gene_name": "Thymidylate synthase",
  "gene_symbol": "TYMS",
  "term_id": "GO:0005829"
}